positive regulation of 'de novo' NAD biosynthetic process from L-tryptophan [GO:1905014] (biological process) Definition: Any process that activates or increases the frequency, rate or extent of 'de novo' NAD biosynthetic process from L-tryptophan. Relationships: is_a GO:0090358; is a type of GO:1900373; is a type of positive regulation of NAD metabolic process [GO:1902690]; is a type of regulation of 'de novo' NAD biosynthetic process from L-tryptophan [GO:1905012]; positively regulates 'de novo' NAD+ biosynthetic process from L-tryptophan [GO:0034354] Sources: GOC:PARL, GOC:TermGenie, GOC:bf, GO_REF:0000058 Also known as: positive regulation of 'de novo' NAD biosynthetic process from tryptophan, up regulation of 'de novo' NAD biosynthetic process from tryptophan, up-regulation of 'de novo' NAD biosynthetic process from tryptophan, upregulation of 'de novo' NAD biosynthetic process from tryptophan, activation of 'de novo' NAD biosynthetic process from tryptophan, activation of de novo NAD biosynthetic process from tryptophan, positive regulation of de novo NAD biosynthetic process from tryptophan, up regulation of de novo NAD biosynthetic process from tryptophan, up-regulation of de novo NAD biosynthetic process from tryptophan, upregulation of de novo NAD biosynthetic process from tryptophan